regulation of chemokine (C-C motif) ligand 20 production [GO:1903884] (biological process) Relationships: is a type of regulation of chemokine production [GO:0032642]; regulates GO:0036392 Subtypes: negative regulation of chemokine (C-C motif) ligand 20 production [GO:1903885], positive regulation of chemokine (C-C motif) ligand 20 production [GO:1903886] References: PMID:20054338 Sources: GOC:TermGenie, GOC:krc, GO_REF:0000058 Definition: Any process that modulates the frequency, rate or extent of chemokine (C-C motif) ligand 20 production. Also known as: regulation of C-C motif chemokine 20 production, regulation of CCL-20 production, regulation of CCL20 production